glycolate transmembrane transporter activity [GO:0043879] (molecular function) Definition: Enables the transfer of glycolate from one side of a membrane to the other. Glycolate is the smallest alpha-hydroxy acid (AHA). Sources: GOC:jl Also known as: glycolic acid transmembrane transporter activity, hydroxyacetic acid transmembrane transporter activity, glcA, glycolate permease Relationships: is a type of monocarboxylic acid transmembrane transporter activity [GO:0008028]; is a type of GO:0015665; is part of glycolate transmembrane transport [GO:0097339]